negative regulation of cutin biosynthetic process [GO:1901958] (biological process) Relationships: is a type of negative regulation of macromolecule biosynthetic process [GO:0010558]; is_a regulation of cutin biosynthetic process [GO:1901957]; RO_0002212 GO:0010143 Also known as: down regulation of cutin anabolism, down regulation of cutin biosynthesis, down regulation of cutin biosynthetic process, down regulation of cutin formation, down regulation of cutin synthesis, down-regulation of cutin anabolism, down-regulation of cutin biosynthesis, down-regulation of cutin biosynthetic process, down-regulation of cutin formation, down-regulation of cutin synthesis, downregulation of cutin anabolism, downregulation of cutin biosynthesis, downregulation of cutin biosynthetic process, downregulation of cutin formation, downregulation of cutin synthesis, inhibition of cutin anabolism, inhibition of cutin biosynthesis, inhibition of cutin formation, inhibition of cutin synthesis, negative regulation of cutin anabolism, negative regulation of cutin biosynthesis, negative regulation of cutin formation, negative regulation of cutin synthesis, inhibition of cutin biosynthetic process Definition: Any process that stops, prevents or reduces the frequency, rate or extent of cutin biosynthetic process. References: PMID:23243127 Sources: GOC:TermGenie, GOC:tb